{
  "gene_symbol": "PRDM15",
  "term_id": "GO:0006357",
  "gene_name": "PR domain zinc finger protein 15",
  "term_label": "regulation of transcription by RNA polymerase II",
  "gene": "UniProtKB:P57071"
}